{
  "term_label": "structural constituent of skin epidermis",
  "gene_symbol": "KRT35",
  "term_id": "GO:0030280",
  "gene_name": "Keratin, type I cuticular Ha5",
  "gene": "UniProtKB:Q92764"
}